L-galactonolactone oxidase activity [GO:0050024] (molecular function) Sources: EC:1.3.3.12, RHEA:20617 Relationships: is a type of GO:0016634; is a type of oxidoreductase activity, acting on the CH-OH group of donors, oxygen as acceptor [GO:0016899] Also known as: L-galactono-1,4-lactone oxidase activity, L-galactono-1,4-lactone:oxygen 3-oxidoreductase activity, L-xylono-1,4-lactone oxidase activity Definition: Catalysis of the reaction: L-galactono-1,4-lactone + O2 = L-ascorbate + H2O2 + H+.